{
  "gene_name": "Sperm protamine P1",
  "gene": "UniProtKB:P04553",
  "gene_symbol": "PRM1",
  "term_label": "Unknown biological process",
  "term_id": "UNKNOWN:0002"
}